mesonephric glomerular mesangium development [GO:0061247] (biological process) Relationships: is a type of GO:0072109; is part of GO:0061231 Definition: The process whose specific outcome is the progression of the mesonephric glomerular mesangium over time, from its formation to the mature structure. The mesonephric glomerular mesangium is the thin membrane connective tissue composed of mesangial cells in the mesonephros, which helps to support the capillary loops in a renal glomerulus. Sources: GOC:mtg_kidney_jan10